{
  "term_label": "odorant binding",
  "gene_symbol": "OR5AR1",
  "gene_name": "Olfactory receptor 5AR1",
  "term_id": "GO:0005549",
  "gene": "UniProtKB:Q8NGP9"
}